{
  "term_id": "UNKNOWN:0003",
  "gene": "UniProtKB:Q8N443",
  "term_label": "Unknown cellular component",
  "gene_symbol": "RIBC1",
  "gene_name": "RIB43A-like with coiled-coils protein 1"
}